{
  "term_id": "GO:0031433",
  "gene_symbol": "MYOZ3",
  "gene_name": "Myozenin-3",
  "gene": "UniProtKB:Q8TDC0",
  "term_label": "telethonin binding"
}